{
  "gene_symbol": "SST",
  "term_id": "UNKNOWN:0001",
  "gene_name": "Somatostatin",
  "gene": "UniProtKB:P61278",
  "term_label": "Unknown molecular function"
}